phenylacetone monooxygenase activity [GO:0033776] (molecular function) Relationships: is a type of oxidoreductase activity, acting on paired donors, with incorporation or reduction of molecular oxygen, NAD(P)H as one donor, and incorporation of one atom of oxygen [GO:0016709] Also known as: PAMO, phenylacetone,NADPH:oxygen oxidoreductase activity Definition: Catalysis of the reaction: H+ + NADPH + O2 + phenylacetone = benzyl acetate + H2O + NADP+. Sources: EC:1.14.13.92, RHEA:10124